neural crest cell differentiation involved in parathyroid gland development [GO:1902638] (biological process) References: PMID:15741317 Sources: GOC:TermGenie, GOC:nhn, GO_REF:0000060 Relationships: is a type of GO:0014033; is part of GO:0060017 Definition: Any neural crest cell differentiation that is involved in parathyroid gland development.